{
  "gene_name": "NLR family pyrin domain-containing protein 2B",
  "gene": "UniProtKB:P0DMW2",
  "gene_symbol": "NLRP2B",
  "term_label": "Unknown molecular function",
  "term_id": "UNKNOWN:0001"
}